{
  "gene": "UniProtKB:O43570",
  "gene_name": "Carbonic anhydrase 12",
  "term_id": "GO:0004089",
  "gene_symbol": "CA12",
  "term_label": "carbonate dehydratase activity"
}